{
  "gene_name": "Homeobox protein Hox-A4",
  "term_id": "GO:0000981",
  "gene": "UniProtKB:Q00056",
  "gene_symbol": "HOXA4",
  "term_label": "DNA-binding transcription factor activity, RNA polymerase II-specific"
}